{
  "term_id": "UNKNOWN:0001",
  "gene": "UniProtKB:Q6PL24",
  "term_label": "Unknown molecular function",
  "gene_symbol": "TMED8",
  "gene_name": "Protein TMED8"
}